{
  "gene": "UniProtKB:Q9BRP0",
  "gene_name": "Transcription factor Ovo-like 2",
  "term_id": "GO:0000978",
  "gene_symbol": "OVOL2",
  "term_label": "RNA polymerase II cis-regulatory region sequence-specific DNA binding"
}